{
  "gene": "UniProtKB:Q9UEF7",
  "gene_symbol": "KL",
  "gene_name": "Klotho",
  "term_label": "fibroblast growth factor receptor binding",
  "term_id": "GO:0005104"
}